{
  "term_label": "central nervous system development",
  "gene_name": "Amyloid beta precursor like protein 2",
  "gene": "UniProtKB:Q06481",
  "term_id": "GO:0007417",
  "gene_symbol": "APLP2"
}